lamellar body membrane [GO:0097232] (cellular component) Definition: The lipid bilayer surrounding a lamellar body. A lamellar body is a membrane-bounded organelle, specialized for the storage and secretion of various substances (surfactant phospholipids, glycoproteins and acid phosphates) which are arranged in the form of tightly packed, concentric, membrane sheets or lamellae. Has some similar properties to, but is distinct from, a lysosome. Subtypes: GO:0097233, epidermal lamellar body membrane [GO:0097234] References: PMID:11940594 Sources: GOC:sl Relationships: is a type of secretory granule membrane [GO:0030667]; is part of lamellar body [GO:0042599]